renal phosphate excretion [GO:0044722] (biological process) Also known as: renal phosphate ion excretion Relationships: is a type of renal tubular secretion [GO:0097254] References: PMID:25287933 Sources: GOC:jl Regulation: RO_0002211 by regulation of renal phosphate excretion [GO:1903402]; negatively regulated by negative regulation of renal phosphate excretion [GO:1903403]; positively regulated by GO:1903404 Definition: The elimination of phosphate ions from peritubular capillaries (or surrounding hemolymph in invertebrates) into the renal tubules to be incorporated subsequently into the urine.